{
  "gene_name": "B-cell lymphoma 3 protein",
  "gene": "UniProtKB:P20749",
  "term_label": "cytosol",
  "term_id": "GO:0005829",
  "gene_symbol": "BCL3"
}